mRNA 3'-UTR AU-rich region binding [GO:0035925] (molecular function) Also known as: adenylate/uridylate-rich element binding, mRNA 3'-UTR adenylate/uridylate-rich element binding, ARE binding, AU-rich element binding Relationships: is a type of mRNA 3'-UTR binding [GO:0003730] References: PMID:31511872, PMID:7892223, PMID:8578590 Sources: GOC:vw Definition: Binding to a region containing frequent adenine and uridine bases within the 3' untranslated region of a mRNA molecule or in pre-mRNA intron. The ARE-binding element consensus is UUAUUUAUU. ARE-binding proteins control the stability and/or translation of mRNAs.